{
  "gene": "UniProtKB:Q8IW75",
  "gene_name": "Serpin A12",
  "term_label": "Unknown biological process",
  "gene_symbol": "SERPINA12",
  "term_id": "UNKNOWN:0002"
}